{
  "gene_name": "DNA polymerase epsilon catalytic subunit A",
  "gene_symbol": "POLE",
  "term_id": "GO:0008622",
  "gene": "UniProtKB:Q07864",
  "term_label": "epsilon DNA polymerase complex"
}